{
  "gene_symbol": "PYM1",
  "gene_name": "Partner of Y14 and mago",
  "gene": "UniProtKB:Q9BRP8",
  "term_id": "GO:0003723",
  "term_label": "RNA binding"
}